{
  "gene_name": "Putative uncharacterized protein LINC02908",
  "term_id": "UNKNOWN:0001",
  "gene": "UniProtKB:Q6ZV77",
  "term_label": "Unknown molecular function",
  "gene_symbol": "LINC02908"
}